{
  "term_label": "P-type sodium:potassium-exchanging transporter activity",
  "gene_name": "Sodium_potassium-transporting ATPase subunit alpha-3",
  "gene_symbol": "ATP1A3",
  "gene": "UniProtKB:P13637",
  "term_id": "GO:0005391"
}